renal vesicle progenitor cell differentiation [GO:0072184] (biological process) Relationships: is a type of cell differentiation involved in kidney development [GO:0061005]; is part of renal vesicle development [GO:0072087] Definition: The process in which relatively unspecialized cells acquire specialized structural and/or functional features that characterize the renal vesicle progenitor cells of the kidney as it progresses from its formation to the mature state. A renal vesicle progenitor cell is a cell that will give rise to terminally differentiated cells of the renal vesicle without self-renewing. Sources: GOC:mtg_kidney_jan10